{
  "gene": "UniProtKB:Q86W24",
  "term_label": "Unknown molecular function",
  "gene_name": "NACHT, LRR and PYD domains-containing protein 14",
  "term_id": "UNKNOWN:0001",
  "gene_symbol": "NLRP14"
}